orcinol 2-monooxygenase activity [GO:0018661] (molecular function) Sources: EC:1.14.13.6, RHEA:19601 Relationships: is_a oxidoreductase activity, acting on paired donors, with incorporation or reduction of molecular oxygen, NAD(P)H as one donor, and incorporation of one atom of oxygen [GO:0016709] Definition: Catalysis of the reaction: H+ + NADH + O2 + orcinol = 2,3,5-trihydroxytoluene + H2O + NAD+. Also known as: orcinol hydroxylase activity, orcinol,NADH:oxygen oxidoreductase (2-hydroxylating)